threonine aldolase activity [GO:0004793] (molecular function) Definition: Catalysis of the reaction: L-threonine = glycine + acetaldehyde. Also known as: L-threonine aldolase activity, L-threonine acetaldehyde-lyase (glycine-forming), L-threonine acetaldehyde-lyase activity Relationships: is a type of aldehyde-lyase activity [GO:0016832] Subtypes: L-allo-threonine aldolase activity [GO:0008732] Sources: RHEA:19625